{
  "gene_symbol": "GSS",
  "gene_name": "Glutathione synthetase",
  "term_id": "GO:0004363",
  "gene": "UniProtKB:P48637",
  "term_label": "glutathione synthase activity"
}